{
  "gene": "UniProtKB:Q8NFA0",
  "term_label": "cysteine-type deubiquitinase activity",
  "term_id": "GO:0004843",
  "gene_name": "Ubiquitin carboxyl-terminal hydrolase 32",
  "gene_symbol": "USP32"
}